{
  "gene_name": "cTAGE family member 6",
  "gene_symbol": "CTAGE6",
  "gene": "UniProtKB:Q86UF2",
  "term_id": "GO:0035459",
  "term_label": "vesicle cargo loading"
}